negative regulation of cardiac muscle myoblast proliferation [GO:0110023] (biological process) Definition: Any process that stops, prevents, or reduces the frequency, rate or extent of cardiac muscle myoblast proliferation. References: PMID:26512644 Sources: GOC:BHF, GOC:BHF_miRNA, GOC:rph Relationships: is a type of regulation of cardiac muscle myoblast proliferation [GO:0110022]; is a type of GO:2000818; negatively regulates cardiac muscle myoblast proliferation [GO:0110021]